{
  "gene": "UniProtKB:Q9UBZ9",
  "term_id": "GO:0070987",
  "gene_name": "DNA repair protein REV1",
  "gene_symbol": "REV1",
  "term_label": "error-free translesion synthesis"
}